{
  "gene_symbol": "GATA3",
  "gene_name": "Trans-acting T-cell-specific transcription factor GATA-3",
  "term_label": "negative regulation of transcription by RNA polymerase II",
  "gene": "UniProtKB:P23771",
  "term_id": "GO:0000122"
}